cellular response to interleukin-6 [GO:0071354] (biological process) Sources: GOC:mah Also known as: cellular response to IL-6 Relationships: is a type of response to interleukin-6 [GO:0070741]; is_a cellular response to cytokine stimulus [GO:0071345] Definition: Any process that results in a change in state or activity of a cell (in terms of movement, secretion, enzyme production, gene expression, etc.) as a result of an interleukin-6 stimulus.